{
  "gene_symbol": "SIGLEC6",
  "term_label": "plasma membrane",
  "gene_name": "Sialic acid-binding Ig-like lectin 6",
  "gene": "UniProtKB:O43699",
  "term_id": "GO:0005886"
}